{
  "term_id": "GO:0008353",
  "gene_name": "Cyclin-dependent kinase 9",
  "gene": "UniProtKB:P50750",
  "gene_symbol": "CDK9",
  "term_label": "RNA polymerase II CTD heptapeptide repeat kinase activity"
}